execution phase of necroptosis [GO:0097528] (biological process) Also known as: necroptosis, execution phase of necroptotic process, necroptotic execution phase References: PMID:20823910 Sources: GOC:mtg_apoptosis Relationships: is a type of cellular process [GO:0009987]; is part of necroptotic process [GO:0070266] Definition: A stage of the necroptotic process that starts after a necroptotic signal has been relayed to the execution machinery. Key steps of the execution phase are swelling of organelles, minor ultrastructural modifications of the nucleus (specifically, dilatation of the nuclear membrane and condensation of chromatin into small, irregular, circumscribed patches) and increased cell volume (oncosis), culminating in the disruption of the plasma membrane and subsequent loss of intracellular contents. The execution phase ends when the cell has died.